{
  "gene": "UniProtKB:P21810",
  "gene_name": "Biglycan",
  "term_id": "UNKNOWN:0001",
  "term_label": "Unknown molecular function",
  "gene_symbol": "BGN"
}